{
  "term_label": "nucleus",
  "gene": "UniProtKB:P45974",
  "gene_name": "Ubiquitin carboxyl-terminal hydrolase 5",
  "term_id": "GO:0005634",
  "gene_symbol": "USP5"
}